{
  "term_label": "cellular response to growth factor stimulus",
  "gene_name": "Activin receptor type-1",
  "gene": "UniProtKB:Q04771",
  "term_id": "GO:0071363",
  "gene_symbol": "ACVR1"
}